{
  "gene": "UniProtKB:Q13601",
  "gene_symbol": "KRR1",
  "term_label": "small-subunit processome",
  "gene_name": "KRR1 small subunit processome component homolog",
  "term_id": "GO:0032040"
}